{
  "gene_symbol": "STK19",
  "gene": "UniProtKB:P49842",
  "gene_name": "Serine_threonine-protein kinase 19",
  "term_label": "Unknown molecular function",
  "term_id": "UNKNOWN:0001"
}